{
  "gene_name": "Olfactory receptor 8H2",
  "gene_symbol": "OR8H2",
  "term_label": "sensory perception of smell",
  "term_id": "GO:0007608",
  "gene": "UniProtKB:Q8N162"
}